{
  "gene": "UniProtKB:Q6ZSY5",
  "gene_symbol": "PPP1R3F",
  "term_label": "protein phosphatase 1 binding",
  "gene_name": "Protein phosphatase 1 regulatory subunit 3F",
  "term_id": "GO:0008157"
}